{
  "gene_symbol": "RIPOR3",
  "gene": "UniProtKB:Q96MK2",
  "term_id": "UNKNOWN:0002",
  "term_label": "Unknown biological process",
  "gene_name": "RIPOR family member 3"
}